carotene biosynthetic process [GO:0016120] (biological process) Subtypes: phytoene biosynthetic process [GO:1901174], lycopene biosynthetic process [GO:1901177], beta-carotene biosynthetic process [GO:1901812], beta-zeacarotene biosynthetic process [GO:1901818], alpha-zeacarotene biosynthetic process [GO:1901821], alpha-carotene biosynthetic process [GO:1901824] Sources: GOC:go_curators Also known as: carotene anabolism, carotene biosynthesis, carotene formation, carotene synthesis Definition: The chemical reactions and pathways resulting in the formation of carotenes, hydrocarbon carotenoids. Relationships: is a type of GO:0016119; is a type of terpene biosynthetic process [GO:0046246]